positive regulation of epithelial cell proliferation involved in wound healing [GO:0060054] (biological process) Definition: Any process that activates or increases the rate or extent of epithelial cell proliferation, contributing to the restoration of integrity to a damaged tissue following an injury. Sources: GOC:dph Relationships: is a type of GO:0050679; is part of wound healing [GO:0042060]